chondroitin 4-sulfotransferase activity [GO:0047756] (molecular function) Definition: Catalysis of the reaction: 3'-phosphoadenosine 5'-phosphosulfate + chondroitin = adenosine 3',5'-bisphosphate + chondroitin 4'-sulfate. Also known as: chondroitin 4-sulphotransferase activity, 3'-phosphoadenylyl-sulfate:chondroitin 4'-sulfotransferase activity Sources: EC:2.8.2.5, MetaCyc:CHONDROITIN-4-SULFOTRANSFERASE-RXN Relationships: is a type of chondroitin sulfotransferase activity [GO:0034481]